{
  "gene_name": "Kelch-like protein 35",
  "term_id": "GO:0005737",
  "gene_symbol": "KLHL35",
  "gene": "UniProtKB:Q6PF15",
  "term_label": "cytoplasm"
}